cardiac conduction [GO:0061337] (biological process) Regulation: RO_0002211 by regulation of cardiac conduction [GO:1903779]; negatively regulated by negative regulation of cardiac conduction [GO:1903780]; positively regulated by positive regulation of cardiac conduction [GO:1903781] Sources: GOC:dph Definition: Transfer of an organized electrical impulse across the heart to coordinate the contraction of cardiac muscles. The process begins with generation of an action potential (in the sinoatrial node (SA) in humans) and ends with a change in the rate, frequency, or extent of the contraction of the heart muscles. Relationships: is a type of regulation of heart contraction [GO:0008016] Subtypes: regulation of heart rate by cardiac conduction [GO:0086091], GO:0086092